{
  "gene_name": "Protein LSM14 homolog B",
  "term_label": "Unknown biological process",
  "gene_symbol": "LSM14B",
  "gene": "UniProtKB:Q9BX40",
  "term_id": "UNKNOWN:0002"
}